{
  "gene": "UniProtKB:Q9BW72",
  "term_id": "UNKNOWN:0001",
  "gene_name": "HIG1 domain family member 2A, mitochondrial",
  "gene_symbol": "HIGD2A",
  "term_label": "Unknown molecular function"
}